cuticle development involved in chitin-based cuticle molting cycle [GO:0042337] (BP) Relationships: is a type of chitin-based cuticle development [GO:0040003]; is part of molting cycle, chitin-based cuticle [GO:0007591] Subtypes: larval chitin-based cuticle development [GO:0008363], pupal chitin-based cuticle development [GO:0008364] Definition: The synthesis and deposition of a chitin-based non-cellular, hardened, or membranous secretion from an epithelial sheet, occurring as part of the molting cycle. An example of this is found in Drosophila melanogaster. Sources: GOC:dph, GOC:jl, GOC:mtg_sensu, GOC:tb Also known as: cuticle anabolism during molting, cuticle biosynthetic process during molting, cuticle formation during molting, cuticle synthesis during molting, chitin-based cuticle development during molting